{
  "term_label": "Unknown biological process",
  "term_id": "UNKNOWN:0002",
  "gene_symbol": "EXOC3L2",
  "gene_name": "Exocyst complex component 3-like protein 2",
  "gene": "UniProtKB:Q2M3D2"
}